{
  "term_label": "sensory organ development",
  "gene_name": "Paired box protein Pax-6",
  "term_id": "GO:0007423",
  "gene_symbol": "PAX6",
  "gene": "UniProtKB:P26367"
}